{
  "gene_symbol": "MMACHC",
  "term_id": "GO:0005737",
  "gene_name": "Cyanocobalamin reductase _ alkylcobalamin dealkylase",
  "gene": "UniProtKB:Q9Y4U1",
  "term_label": "cytoplasm"
}